{
  "gene_name": "Potassium voltage-gated channel subfamily A member 5",
  "gene_symbol": "KCNA5",
  "term_label": "intercalated disc",
  "term_id": "GO:0014704",
  "gene": "UniProtKB:P22460"
}